{
  "gene": "UniProtKB:P42575",
  "term_id": "GO:0006915",
  "term_label": "apoptotic process",
  "gene_name": "Caspase-2",
  "gene_symbol": "CASP2"
}